{
  "gene_name": "Homeobox protein CDX-1",
  "gene": "UniProtKB:P47902",
  "gene_symbol": "CDX1",
  "term_label": "anterior/posterior axis specification",
  "term_id": "GO:0009948"
}